{
  "term_id": "GO:0061630",
  "gene": "UniProtKB:Q96P09",
  "term_label": "ubiquitin protein ligase activity",
  "gene_name": "Baculoviral IAP repeat-containing protein 8",
  "gene_symbol": "BIRC8"
}